{
  "gene": "UniProtKB:Q15018",
  "term_id": "GO:0008608",
  "gene_name": "BRISC complex subunit Abraxas 2",
  "term_label": "attachment of spindle microtubules to kinetochore",
  "gene_symbol": "ABRAXAS2"
}